{
  "gene": "UniProtKB:Q9NP91",
  "term_id": "GO:1903804",
  "gene_symbol": "SLC6A20",
  "term_label": "glycine import across plasma membrane",
  "gene_name": "Sodium- and chloride-dependent transporter XTRP3"
}